{
  "gene_name": "Paired box protein Pax-9",
  "term_label": "regulation of transcription by RNA polymerase II",
  "gene_symbol": "PAX9",
  "term_id": "GO:0006357",
  "gene": "UniProtKB:P55771"
}